{
  "gene_name": "Inactive serine protease PAMR1",
  "gene": "UniProtKB:Q6UXH9",
  "term_id": "UNKNOWN:0001",
  "gene_symbol": "PAMR1",
  "term_label": "Unknown molecular function"
}